{
  "gene_symbol": "IGLV3-32",
  "term_label": "immunoglobulin complex",
  "term_id": "GO:0019814",
  "gene_name": "Probable non-functional immunoglobulin lambda variable 3-32",
  "gene": "UniProtKB:A0A0A0MS00"
}